negative regulation of synaptic transmission [GO:0050805] (biological process) Also known as: down regulation of synaptic transmission, down-regulation of synaptic transmission, downregulation of synaptic transmission, inhibition of synaptic transmission Definition: Any process that stops, prevents, or reduces the frequency, rate or extent of synaptic transmission, the process of communication from a neuron to a target (neuron, muscle, or secretory cell) across a synapse. Sources: GOC:ai Subtypes: negative regulation of synaptic transmission, cholinergic [GO:0032223], GO:0032227, negative regulation of synaptic transmission, GABAergic [GO:0032229], negative regulation of synaptic transmission, glutamatergic [GO:0051967], negative regulation of synaptic transmission, glycinergic [GO:0060093], long-term synaptic depression [GO:0060292], negative regulation of neuromuscular synaptic transmission [GO:1900074] Relationships: is a type of negative regulation of cell communication [GO:0010648]; is a type of negative regulation of signaling [GO:0023057]; is a type of modulation of chemical synaptic transmission [GO:0050804]; negatively regulates chemical synaptic transmission [GO:0007268]